{
  "gene_name": "Osteopontin",
  "gene_symbol": "SPP1",
  "term_id": "GO:0001649",
  "term_label": "osteoblast differentiation",
  "gene": "UniProtKB:P10451"
}